{
  "gene": "UniProtKB:Q9NTN9",
  "term_id": "GO:0045499",
  "gene_name": "Semaphorin-4G",
  "gene_symbol": "SEMA4G",
  "term_label": "chemorepellent activity"
}